{
  "gene_name": "T-box transcription factor TBX10",
  "term_id": "GO:0006357",
  "gene": "UniProtKB:O75333",
  "term_label": "regulation of transcription by RNA polymerase II",
  "gene_symbol": "TBX10"
}